{
  "term_label": "mitochondrion",
  "gene": "UniProtKB:Q96BP2",
  "gene_symbol": "CHCHD1",
  "term_id": "GO:0005739",
  "gene_name": "Small ribosomal subunit protein mS37"
}